{
  "term_label": "RNA polymerase II transcription regulatory region sequence-specific DNA binding",
  "gene_name": "Zinc finger protein 441",
  "gene": "UniProtKB:Q8N8Z8",
  "term_id": "GO:0000977",
  "gene_symbol": "ZNF441"
}